somatic diversification of immunoglobulins involved in immune response [GO:0002208] (biological process) Also known as: somatic diversification of antibodies during immune response, somatic diversification of immunoglobulins during immune response Relationships: is a type of GO:0016445; is part of immunoglobulin production involved in immunoglobulin-mediated immune response [GO:0002381] Subtypes: somatic recombination of immunoglobulin genes involved in immune response [GO:0002204], GO:0002205, gene conversion of immunoglobulin genes involved in immune response [GO:0002207] Definition: The somatic process that results in the generation of sequence diversity of immunoglobulins after induction, and contributes to an immune response. References: PMID:14991701 Sources: GOC:add, ISBN:0781735149